{
  "gene_symbol": "WDR53",
  "gene": "UniProtKB:Q7Z5U6",
  "gene_name": "WD repeat-containing protein 53",
  "term_label": "Unknown biological process",
  "term_id": "UNKNOWN:0002"
}